{
  "term_id": "GO:0045892",
  "gene": "UniProtKB:Q8N6I1",
  "gene_symbol": "EID2",
  "gene_name": "EP300-interacting inhibitor of differentiation 2",
  "term_label": "negative regulation of DNA-templated transcription"
}